{
  "gene": "UniProtKB:Q06609",
  "gene_name": "DNA repair protein RAD51 homolog 1",
  "term_label": "condensed nuclear chromosome",
  "gene_symbol": "RAD51",
  "term_id": "GO:0000794"
}